{
  "gene_symbol": "RPL12",
  "gene": "UniProtKB:P30050",
  "term_label": "structural constituent of ribosome",
  "gene_name": "Large ribosomal subunit protein uL11",
  "term_id": "GO:0003735"
}